{
  "gene": "UniProtKB:P50583",
  "term_id": "GO:0006754",
  "gene_name": "Bis(5'-nucleosyl)-tetraphosphatase [asymmetrical]",
  "gene_symbol": "NUDT2",
  "term_label": "ATP biosynthetic process"
}